{
  "term_id": "GO:0005769",
  "gene_symbol": "WASH2P",
  "gene": "UniProtKB:Q6VEQ5",
  "gene_name": "WAS protein family homolog 2",
  "term_label": "early endosome"
}